{
  "gene_name": "Protein arginine N-methyltransferase 8",
  "term_label": "histone methyltransferase activity",
  "gene": "UniProtKB:Q9NR22",
  "term_id": "GO:0042054",
  "gene_symbol": "PRMT8"
}